negative regulation of tubulin deacetylation [GO:1904428] (biological process) References: PMID:23886946 Sources: GOC:TermGenie, GO_REF:0000058 Relationships: is a type of GO:0031400; is a type of regulation of tubulin deacetylation [GO:0090043]; negatively regulates GO:0090042 Definition: Any process that stops, prevents or reduces the frequency, rate or extent of tubulin deacetylation. Also known as: down regulation of tubulin deacetylation, down-regulation of tubulin deacetylation, downregulation of tubulin deacetylation, inhibition of tubulin deacetylation